{
  "gene": "UniProtKB:O95859",
  "term_id": "UNKNOWN:0001",
  "term_label": "Unknown molecular function",
  "gene_symbol": "TSPAN12",
  "gene_name": "Tetraspanin-12"
}